{
  "gene_name": "Keratin, type II cuticular Hb1",
  "term_id": "GO:0045109",
  "gene": "UniProtKB:Q14533",
  "gene_symbol": "KRT81",
  "term_label": "intermediate filament organization"
}